{
  "gene": "UniProtKB:P10914",
  "term_id": "GO:0000978",
  "term_label": "RNA polymerase II cis-regulatory region sequence-specific DNA binding",
  "gene_name": "Interferon regulatory factor 1",
  "gene_symbol": "IRF1"
}